{
  "gene_name": "KRAB domain-containing protein 1",
  "gene": "UniProtKB:C9JBD0",
  "gene_symbol": "KRBOX1",
  "term_label": "RNA polymerase II cis-regulatory region sequence-specific DNA binding",
  "term_id": "GO:0000978"
}